{
  "term_label": "regulation of DNA-templated transcription",
  "gene": "UniProtKB:Q9NQV8",
  "gene_name": "PR domain zinc finger protein 8",
  "gene_symbol": "PRDM8",
  "term_id": "GO:0006355"
}